{
  "term_id": "GO:0004360",
  "gene_symbol": "GFPT2",
  "term_label": "glutamine-fructose-6-phosphate transaminase (isomerizing) activity",
  "gene": "UniProtKB:O94808",
  "gene_name": "Glutamine--fructose-6-phosphate aminotransferase [isomerizing] 2"
}